{
  "gene_symbol": "CDH16",
  "term_label": "cell adhesion molecule binding",
  "gene": "UniProtKB:O75309",
  "gene_name": "Cadherin-16",
  "term_id": "GO:0050839"
}